regulation of protein localization to cell cortex [GO:1904776] (biological process) Also known as: regulation of protein localisation to cell cortex Note: An example is cye-1 in C. elegans, UniProt ID O01501 in PMID:17115027. Relationships: is a type of regulation of protein localization to cell periphery [GO:1904375]; regulates protein localization to cell cortex [GO:0072697] Subtypes: regulation of protein localization to medial cortex [GO:0106011], GO:1904370, GO:1904777, GO:1904778, regulation of protein localization to cell cortex of cell tip [GO:1990895] Definition: Any process that modulates the frequency, rate or extent of protein localization to cell cortex. References: PMID:17115027 Sources: GOC:TermGenie, GO_REF:0000058